{
  "gene_symbol": "F13A1",
  "term_id": "GO:0072378",
  "gene": "UniProtKB:P00488",
  "term_label": "blood coagulation, fibrin clot formation",
  "gene_name": "Coagulation factor XIII A chain"
}